{
  "gene_symbol": "CLASP1",
  "term_label": "kinetochore",
  "gene_name": "CLIP-associating protein 1",
  "term_id": "GO:0000776",
  "gene": "UniProtKB:Q7Z460"
}